{
  "gene": "UniProtKB:Q0VDD7",
  "term_label": "Unknown biological process",
  "gene_symbol": "BRME1",
  "term_id": "UNKNOWN:0002",
  "gene_name": "Break repair meiotic recombinase recruitment factor 1"
}